FACT complex binding [GO:0062059] (molecular function) References: PMID:10682845 Definition: Binding to a FACT complex. Relationships: is a type of protein-containing complex binding [GO:0044877]